{
  "term_label": "leading strand elongation",
  "gene_symbol": "POLE3",
  "gene_name": "DNA polymerase epsilon subunit 3",
  "term_id": "GO:0006272",
  "gene": "UniProtKB:Q9NRF9"
}